17-methylnonadec-1-ene metabolic process [GO:1900882] (biological process) Definition: The chemical reactions and pathways involving 17-methylnonadec-1-ene. Sources: GOC:TermGenie, GOC:mengo_curators Also known as: 17-methylnonadec-1-ene metabolism Relationships: is a type of GO:1900673 Subtypes: GO:1900883